{
  "term_id": "GO:0007155",
  "gene": "UniProtKB:Q9Y5H9",
  "gene_name": "Protocadherin alpha-2",
  "gene_symbol": "PCDHA2",
  "term_label": "cell adhesion"
}